{
  "term_id": "GO:0009653",
  "gene_name": "Forkhead box protein I3",
  "gene_symbol": "FOXI3",
  "term_label": "anatomical structure morphogenesis",
  "gene": "UniProtKB:A8MTJ6"
}